positive regulation of type IIb hypersensitivity [GO:0001801] (BP) Also known as: up regulation of type IIb hypersensitivity, up-regulation of type IIb hypersensitivity, upregulation of type IIb hypersensitivity, activation of type IIb hypersensitivity, stimulation of type IIb hypersensitivity Definition: Any process that activates or increases the frequency, rate or extent of type IIb hypersensitivity, a type of inflammatory response. Sources: GOC:add, ISBN:0781735149 Relationships: is_a regulation of type IIb hypersensitivity [GO:0001799]; is a type of positive regulation of type II hypersensitivity [GO:0002894]; positively regulates type IIb hypersensitivity [GO:0001795]